actin polymerization or depolymerization [GO:0008154] (biological process) Definition: Assembly or disassembly of actin filaments by the addition or removal of actin monomers from a filament. Sources: GOC:mah Relationships: is a type of actin filament organization [GO:0007015] Subtypes: actin filament polymerization [GO:0030041], actin filament depolymerization [GO:0030042] Regulation: regulated by GO:0008064